cell cortex region [GO:0099738] (cellular component) Definition: The complete extent of cell cortex that underlies some some region of the plasma membrane. Sources: GOC:dos Also known as: perimembrane region Relationships: is a type of cell cortex [GO:0005938]; is a type of cytoplasmic region [GO:0099568]; is part of cell cortex [GO:0005938] Subtypes: GO:0031097, apical cortex [GO:0045179], basal cortex [GO:0045180], cell cortex of cell tip [GO:0051285], anterior cell cortex [GO:0061802], posterior cell cortex [GO:0061803], lateral cell cortex [GO:0097575], presynaptic active zone cytoplasmic component [GO:0098831], presynaptic endocytic zone cytoplasmic component [GO:0098834], postsynaptic endocytic zone cytoplasmic component [GO:0099631], cell leading edge cell cortex [GO:1904269], equatorial cell cortex [GO:1990753]